{
  "gene_name": "MORF4 family-associated protein 1-like 1",
  "gene_symbol": "MRFAP1L1",
  "term_label": "Unknown molecular function",
  "gene": "UniProtKB:Q96HT8",
  "term_id": "UNKNOWN:0001"
}